{
  "gene_name": "PHD finger protein 21A",
  "gene_symbol": "PHF21A",
  "term_label": "chromatin binding",
  "term_id": "GO:0003682",
  "gene": "UniProtKB:Q96BD5"
}